{
  "gene_name": "Eukaryotic elongation factor 2 kinase",
  "gene": "UniProtKB:O00418",
  "term_label": "elongation factor-2 kinase activity",
  "gene_symbol": "EEF2K",
  "term_id": "GO:0004686"
}